formate efflux transmembrane transporter activity [GO:0015660] (molecular function) Relationships: is a type of formate transmembrane transporter activity [GO:0015499]; is a type of efflux transmembrane transporter activity [GO:0015562] Also known as: formate efflux permease activity Definition: Enables the transfer of formate from the inside of the cell to the outside of the cell across a membrane. Sources: GOC:mtg_transport, ISBN:0815340729